{
  "gene_symbol": "PTGES3L",
  "term_label": "chaperone-mediated protein complex assembly",
  "gene": "UniProtKB:E9PB15",
  "gene_name": "Putative protein PTGES3L",
  "term_id": "GO:0051131"
}